{
  "gene_name": "Olfactory receptor 4D5",
  "gene": "UniProtKB:Q8NGN0",
  "gene_symbol": "OR4D5",
  "term_label": "plasma membrane",
  "term_id": "GO:0005886"
}